cellular response to amyloid-beta [GO:1904646] (BP) References: PMID:23555824 Sources: GOC:TermGenie, GO_REF:0000071 Also known as: cellular response to beta-amyloid, cellular response to beta-amyloids Relationships: is a type of cellular response to nitrogen compound [GO:1901699]; is a type of GO:1901701; is a type of GO:1904645 Definition: Any process that results in a change in state or activity of a cell (in terms of movement, secretion, enzyme production, gene expression, etc.) as a result of a amyloid-beta stimulus.